{
  "gene": "UniProtKB:P15812",
  "term_id": "GO:0001916",
  "gene_symbol": "CD1E",
  "gene_name": "T-cell surface glycoprotein CD1e, membrane-associated",
  "term_label": "positive regulation of T cell mediated cytotoxicity"
}